regulation of nitric oxide metabolic process [GO:0080164] (biological process) Sources: GOC:DHL Definition: Any process that modulates the frequency, rate or extent of the chemical reactions and pathways involving nitric oxide, nitrogen monoxide (NO), a colorless gas only slightly soluble in water. Relationships: is a type of regulation of metabolic process [GO:0019222]; regulates nitric oxide metabolic process [GO:0046209] Subtypes: regulation of nitric oxide biosynthetic process [GO:0045428]